{
  "gene_name": "Probable G-protein coupled receptor 179",
  "term_label": "Unknown cellular component",
  "term_id": "UNKNOWN:0003",
  "gene": "UniProtKB:Q6PRD1",
  "gene_symbol": "GPR179"
}